{
  "term_id": "GO:0005923",
  "gene_symbol": "OCLN",
  "term_label": "bicellular tight junction",
  "gene_name": "Occludin",
  "gene": "UniProtKB:Q16625"
}